{
  "term_label": "L-phenylalanine catabolic process",
  "gene_name": "Dihydropteridine reductase",
  "gene": "UniProtKB:P09417",
  "gene_symbol": "QDPR",
  "term_id": "GO:0006559"
}